{
  "term_label": "metalloendopeptidase activity",
  "gene_name": "A disintegrin and metalloproteinase with thrombospondin motifs 8",
  "gene": "UniProtKB:Q9UP79",
  "gene_symbol": "ADAMTS8",
  "term_id": "GO:0004222"
}